{
  "gene_name": "Ras and Rab interactor 3",
  "term_label": "Unknown biological process",
  "term_id": "UNKNOWN:0002",
  "gene": "UniProtKB:Q8TB24",
  "gene_symbol": "RIN3"
}